{
  "gene_symbol": "ATP5F1A",
  "gene": "UniProtKB:P25705",
  "term_id": "GO:0045259",
  "term_label": "proton-transporting ATP synthase complex",
  "gene_name": "ATP synthase subunit alpha, mitochondrial"
}